{
  "term_id": "GO:0045109",
  "gene_symbol": "KRT37",
  "gene_name": "Keratin, type I cuticular Ha7",
  "term_label": "intermediate filament organization",
  "gene": "UniProtKB:O76014"
}